{
  "gene_symbol": "LRRC10B",
  "term_id": "UNKNOWN:0002",
  "gene_name": "Leucine-rich repeat-containing protein 10B",
  "term_label": "Unknown biological process",
  "gene": "UniProtKB:A6NIK2"
}